{
  "term_label": "positive regulation of pseudopodium assembly",
  "gene_name": "Cdc42 effector protein 4",
  "term_id": "GO:0031274",
  "gene": "UniProtKB:Q9H3Q1",
  "gene_symbol": "CDC42EP4"
}